{
  "term_id": "GO:0005634",
  "gene_symbol": "ANP32E",
  "gene": "UniProtKB:Q9BTT0",
  "term_label": "nucleus",
  "gene_name": "Acidic leucine-rich nuclear phosphoprotein 32 family member E"
}